{
  "gene_symbol": "CA3",
  "term_id": "UNKNOWN:0002",
  "gene": "UniProtKB:P07451",
  "term_label": "Unknown biological process",
  "gene_name": "Carbonic anhydrase 3"
}